{
  "gene_name": "Isocitrate dehydrogenase [NADP], mitochondrial",
  "term_label": "isocitrate dehydrogenase (NADP+) activity",
  "gene_symbol": "IDH2",
  "term_id": "GO:0004450",
  "gene": "UniProtKB:P48735"
}